{
  "gene_symbol": "RXRG",
  "term_id": "GO:0048384",
  "gene_name": "Retinoic acid receptor RXR-gamma",
  "term_label": "retinoic acid receptor signaling pathway",
  "gene": "UniProtKB:P48443"
}